{
  "gene": "UniProtKB:Q9GZM8",
  "term_id": "GO:0016477",
  "gene_symbol": "NDEL1",
  "term_label": "cell migration",
  "gene_name": "Nuclear distribution protein nudE-like 1"
}